{
  "gene": "UniProtKB:P49841",
  "term_label": "tau-protein kinase activity",
  "gene_name": "Glycogen synthase kinase-3 beta",
  "gene_symbol": "GSK3B",
  "term_id": "GO:0050321"
}